{
  "gene": "UniProtKB:Q8N3R9",
  "gene_name": "Protein PALS1",
  "term_id": "GO:0045197",
  "term_label": "establishment or maintenance of epithelial cell apical/basal polarity",
  "gene_symbol": "PALS1"
}